{
  "gene_symbol": "RC3H2",
  "gene_name": "Roquin-2",
  "term_label": "ubiquitin protein ligase activity",
  "gene": "UniProtKB:Q9HBD1",
  "term_id": "GO:0061630"
}